{
  "term_label": "Unknown molecular function",
  "term_id": "UNKNOWN:0001",
  "gene_name": "T cell receptor alpha joining 47 (Fragment)",
  "gene": "UniProtKB:A0A075B6Y5",
  "gene_symbol": "TRAJ47"
}